{
  "gene_symbol": "IRF1",
  "gene": "UniProtKB:P10914",
  "term_id": "GO:0002376",
  "term_label": "immune system process",
  "gene_name": "Interferon regulatory factor 1"
}